{
  "gene_symbol": "TTYH3",
  "gene_name": "Protein tweety homolog 3",
  "term_label": "volume-sensitive chloride channel activity",
  "gene": "UniProtKB:Q9C0H2",
  "term_id": "GO:0072320"
}